establishment of epithelial cell apical/basal polarity involved in camera-type eye morphogenesis [GO:0003412] (biological process) Relationships: is a type of establishment of epithelial cell apical/basal polarity [GO:0045198]; is part of camera-type eye morphogenesis [GO:0048593] Sources: GOC:ascb_2009, GOC:dph, GOC:tb Definition: The specification and formation of the apicobasal polarity of an epithelial cell that contributes to the shaping of a camera-type eye.